{
  "term_id": "GO:0005737",
  "term_label": "cytoplasm",
  "gene_symbol": "TRIM22",
  "gene": "UniProtKB:Q8IYM9",
  "gene_name": "E3 ubiquitin-protein ligase TRIM22"
}